P-type cadmium transporter activity [GO:0008551] (molecular function) References: PMID:17326661 Definition: Enables the transfer of a solute or solutes from one side of a membrane to the other according to the reaction: ATP + H2O + Cd2+(in) = ADP + phosphate + Cd2+(out). Also known as: cadmium exporting ATPase activity, cadmium-translocating P-type ATPase activity, cadmium-exporting ATPase activity, Cd(2+)-exporting ATPase activity, Cd2+-exporting ATPase activity, cadmium transmembrane transporter activity, phosphorylative mechanism Relationships: is a type of GO:0015086; is a type of GO:0015662; is a type of ATPase-coupled monoatomic cation transmembrane transporter activity [GO:0019829]